pyruvate, water dikinase activity [GO:0008986] (MF) Definition: Catalysis of the reaction: ATP + H2O + pyruvate = AMP + 2 H+ + phosphate + phosphoenolpyruvate. Sources: RHEA:11364 Also known as: PEP synthase activity, water pyruvate dikinase activity, ATP:pyruvate, water phosphotransferase activity, PEP synthetase activity, phoephoenolpyruvate synthetase activity, phosphoenolpyruvate synthase activity, phosphoenolpyruvic synthase activity, phosphopyruvate synthetase activity, pyruvate,water dikinase activity, pyruvate-water dikinase (phosphorylating) Relationships: is a type of kinase activity [GO:0016301]; is a type of phosphotransferase activity, paired acceptors [GO:0016781]